{
  "term_id": "UNKNOWN:0002",
  "gene_name": "Endogenous retrovirus group K member 113 Env polyprotein",
  "term_label": "Unknown biological process",
  "gene": "UniProtKB:Q902F9",
  "gene_symbol": "HERVK_113"
}